{
  "gene": "UniProtKB:Q96NN9",
  "term_label": "oxidoreductase activity, acting on NAD(P)H",
  "gene_symbol": "AIFM3",
  "term_id": "GO:0016651",
  "gene_name": "Apoptosis-inducing factor 3"
}